{
  "gene": "UniProtKB:O95793",
  "gene_name": "Double-stranded RNA-binding protein Staufen homolog 1",
  "gene_symbol": "STAU1",
  "term_id": "GO:0043005",
  "term_label": "neuron projection"
}